{
  "gene": "UniProtKB:Q86UU1",
  "gene_name": "Pleckstrin homology-like domain family B member 1",
  "term_label": "basement membrane organization",
  "gene_symbol": "PHLDB1",
  "term_id": "GO:0071711"
}